{
  "gene_symbol": "DFFA",
  "gene": "UniProtKB:O00273",
  "term_id": "GO:1900118",
  "gene_name": "DNA fragmentation factor subunit alpha",
  "term_label": "negative regulation of execution phase of apoptosis"
}